{
  "term_label": "regulation of glycogen biosynthetic process",
  "gene": "UniProtKB:Q6ZSY5",
  "gene_name": "Protein phosphatase 1 regulatory subunit 3F",
  "term_id": "GO:0005979",
  "gene_symbol": "PPP1R3F"
}